{
  "gene_symbol": "KIF15",
  "gene_name": "Kinesin-like protein KIF15",
  "gene": "UniProtKB:Q9NS87",
  "term_label": "kinesin complex",
  "term_id": "GO:0005871"
}